{
  "term_id": "GO:0015695",
  "gene_symbol": "SLC22A2",
  "gene_name": "Solute carrier family 22 member 2",
  "term_label": "organic cation transport",
  "gene": "UniProtKB:O15244"
}